positive regulation of organelle organization [GO:0010638] (biological process) Definition: Any process that increases the frequency, rate or extent of a process involved in the formation, arrangement of constituent parts, or disassembly of an organelle. Subtypes: GO:0010636, positive regulation of vesicle fusion [GO:0031340], GO:0044090, positive regulation of spermatid nuclear differentiation [GO:0045702], positive regulation of cytoskeleton organization [GO:0051495], positive regulation of nuclear division [GO:0051785], positive regulation of mitochondrial fission [GO:0090141], GO:0090200, GO:1900064, GO:1901030, positive regulation of autophagosome maturation [GO:1901098], positive regulation of mitochondrial DNA metabolic process [GO:1901860], positive regulation of organelle assembly [GO:1902117], positive regulation of melanosome organization [GO:1903058], positive regulation of endoplasmic reticulum tubular network organization [GO:1903373], positive regulation of protein insertion into mitochondrial outer membrane [GO:1903638], positive regulation of cristae formation [GO:1903852], GO:1904411, positive regulation of endosome organization [GO:1904980], positive regulation of phagosome maturation [GO:1905164], GO:1905194, GO:1905798, positive regulation of postsynaptic density organization [GO:1905876], GO:2001252 Also known as: positive regulation of organelle organisation, positive regulation of organelle organization and biogenesis Sources: GOC:dph, GOC:tb Relationships: is a type of regulation of organelle organization [GO:0033043]; is a type of GO:0051130; positively regulates organelle organization [GO:0006996]